{
  "term_id": "GO:0071364",
  "gene_symbol": "GAREM1",
  "gene_name": "GRB2-associated and regulator of MAPK protein 1",
  "term_label": "cellular response to epidermal growth factor stimulus",
  "gene": "UniProtKB:Q9H706"
}